{
  "term_label": "Unknown cellular component",
  "gene_name": "Olfactory receptor 5AL1",
  "gene_symbol": "OR5AL1",
  "term_id": "UNKNOWN:0003",
  "gene": "UniProtKB:P0C617"
}